{
  "gene_name": "Translocation protein SEC62",
  "term_label": "endoplasmic reticulum",
  "term_id": "GO:0005783",
  "gene_symbol": "SEC62",
  "gene": "UniProtKB:Q99442"
}